{
  "term_label": "RNA polymerase II cis-regulatory region sequence-specific DNA binding",
  "gene_name": "Fez family zinc finger protein 1",
  "gene": "UniProtKB:A0PJY2",
  "gene_symbol": "FEZF1",
  "term_id": "GO:0000978"
}